{
  "gene": "UniProtKB:P17010",
  "term_label": "nucleus",
  "gene_symbol": "ZFX",
  "gene_name": "Zinc finger X-chromosomal protein",
  "term_id": "GO:0005634"
}